{
  "gene_name": "Parathyroid hormone-related protein",
  "gene": "UniProtKB:P12272",
  "term_label": "peptide hormone receptor binding",
  "gene_symbol": "PTHLH",
  "term_id": "GO:0051428"
}